{
  "term_label": "Unknown cellular component",
  "gene_name": "Transcription cofactor vestigial-like protein 4",
  "gene": "UniProtKB:Q14135",
  "term_id": "UNKNOWN:0003",
  "gene_symbol": "VGLL4"
}